{
  "gene_symbol": "ARHGAP15",
  "term_label": "cytoplasm",
  "term_id": "GO:0005737",
  "gene": "UniProtKB:Q53QZ3",
  "gene_name": "Rho GTPase-activating protein 15"
}